{
  "term_label": "intracellular signal transduction",
  "gene_name": "Serine_threonine-protein kinase 4",
  "term_id": "GO:0035556",
  "gene_symbol": "STK4",
  "gene": "UniProtKB:Q13043"
}